amidase activity [GO:0004040] (molecular function) Also known as: acetamidase activity, N-acetylaminohydrolase activity, acylamidase activity, acylamide amidohydrolase activity, acylase activity, amidohydrolase activity, fatty acylamidase activity Definition: Catalysis of the reaction: a monocarboxylic acid amide + H2O = a monocarboxylate + NH4+. Sources: RHEA:12020 Relationships: is a type of hydrolase activity, acting on carbon-nitrogen (but not peptide) bonds, in linear amides [GO:0016811] Subtypes: GO:0004067, GO:0004328, nicotinamidase activity [GO:0008936], indoleacetamide hydrolase activity [GO:0043864]